{
  "term_id": "GO:0005634",
  "term_label": "nucleus",
  "gene_symbol": "ZNF3",
  "gene": "UniProtKB:P17036",
  "gene_name": "Zinc finger protein 3"
}